{
  "term_label": "mitochondrion",
  "gene_name": "Isocitrate dehydrogenase [NADP], mitochondrial",
  "gene_symbol": "IDH2",
  "term_id": "GO:0005739",
  "gene": "UniProtKB:P48735"
}